{
  "term_id": "GO:0019814",
  "gene": "UniProtKB:A0A0B4J264",
  "term_label": "immunoglobulin complex",
  "gene_name": "T cell receptor alpha variable 38-1",
  "gene_symbol": "TRAV38-1"
}